induction of conjugation with cellular fusion [GO:0010514] (biological process) Definition: The process in which a cell initiates conjugation with cellular fusion. Conjugation with cellular fusion is the process that results in the union of cellular and genetic information from compatible mating types. Relationships: is a type of positive regulation of conjugation with cellular fusion [GO:0031139] Regulation: negatively regulated by negative regulation of induction of conjugation with cellular fusion [GO:0010515]; positively regulated by positive regulation of induction of conjugation with cellular fusion [GO:1900237] Subtypes: GO:0031140 Sources: GOC:dph, GOC:tb